{
  "gene": "UniProtKB:P18405",
  "gene_name": "3-oxo-5-alpha-steroid 4-dehydrogenase 1",
  "gene_symbol": "SRD5A1",
  "term_id": "GO:0006702",
  "term_label": "androgen biosynthetic process"
}